anthocyanin-containing compound metabolic process [GO:0046283] (biological process) Regulation: regulated by regulation of anthocyanin metabolic process [GO:0031537]; negatively regulated by negative regulation of anthocyanin metabolic process [GO:0031538]; positively regulated by positive regulation of anthocyanin metabolic process [GO:0031539] Definition: The chemical reactions and pathways involving anthocyanins, any member of a group of intensely colored soluble glycosides of anthocyanidins that occur in plants. They are responsible from most of the scarlet, purple, mauve and blue coloring in higher plants, especially of flowers. Also known as: anthocyanin metabolic process, anthocyanin metabolism Sources: ISBN:0198506732 Subtypes: anthocyanin-containing compound biosynthetic process [GO:0009718], anthocyanin-containing compound catabolic process [GO:0046284] Relationships: is a type of flavonoid metabolic process [GO:0009812]; is a type of pigment metabolic process [GO:0042440]